cytolysis in another organism [GO:0051715] (biological process) Also known as: cytolysis in other organism, cytolysis of cells of another organism, envenomation resulting in cytolysis in another organism, envenomation resulting in cytolysis in other organism Definition: The killing by an organism of a cell in another organism by means of the rupture of cell membranes and the loss of cytoplasm. Relationships: is a type of cytolysis [GO:0019835]; is a type of killing of cells of another organism [GO:0031640] Subtypes: symbiont-mediated cytolysis of host cell [GO:0001897], hemolysis in another organism [GO:0044179] References: PMID:22484288 Sources: GOC:ai